mast cell chemotaxis [GO:0002551] (biological process) Definition: The movement of a mast cell in response to an external stimulus. Relationships: is a type of leukocyte chemotaxis [GO:0030595]; is a type of mast cell migration [GO:0097531] Regulation: regulated by regulation of mast cell chemotaxis [GO:0060753]; positively regulated by positive regulation of mast cell chemotaxis [GO:0060754]; negatively regulated by negative regulation of mast cell chemotaxis [GO:0060755] References: PMID:11292027, PMID:12789214, PMID:16448392 Sources: GOC:add